SCF-Dia2/Pof3 ubiquitin ligase complex [GO:0097663] (cellular component) References: PMID:14747994, PMID:15147268 Sources: GOC:jd, GOC:vw Relationships: is a type of SCF ubiquitin ligase complex [GO:0019005] Definition: An SCF ubiquitin ligase complex in which the F-box protein is Dia2 in S. cerevisiae (Pof3 in S. pombe).